{
  "gene_symbol": "KIFC1",
  "gene": "UniProtKB:Q9BW19",
  "term_label": "kinesin complex",
  "term_id": "GO:0005871",
  "gene_name": "Kinesin-like protein KIFC1"
}